{
  "term_label": "Unknown biological process",
  "gene_symbol": "DDAH2",
  "gene": "UniProtKB:O95865",
  "gene_name": "N(G),N(G)-dimethylarginine dimethylaminohydrolase 2",
  "term_id": "UNKNOWN:0002"
}